positive regulation of response to DNA damage checkpoint signaling [GO:1902154] (biological process) Subtypes: positive regulation of response to G1 DNA damage checkpoint signaling [GO:1902156], positive regulation of response to G2 DNA damage checkpoint signaling [GO:1902158] Also known as: activation of DNA damage checkpoint effector process, activation of response to signal involved in DNA damage checkpoint, positive regulation of DNA damage checkpoint effector process, positive regulation of response to signal involved in DNA damage checkpoint, up regulation of DNA damage checkpoint effector process, up regulation of response to DNA damage checkpoint signaling, up regulation of response to signal involved in DNA damage checkpoint, up-regulation of DNA damage checkpoint effector process, up-regulation of response to DNA damage checkpoint signaling, up-regulation of response to signal involved in DNA damage checkpoint, upregulation of DNA damage checkpoint effector process, upregulation of response to DNA damage checkpoint signaling, upregulation of response to signal involved in DNA damage checkpoint, activation of response to DNA damage checkpoint signaling Definition: Any process that activates or increases the frequency, rate or extent of response to DNA damage checkpoint signaling. Sources: GOC:TermGenie, GOC:mtg_cell_cycle Relationships: is a type of positive regulation of response to DNA integrity checkpoint signaling [GO:1902152]; is_a regulation of response to DNA damage checkpoint signaling [GO:1902153]; positively regulates GO:0072423